{
  "gene": "UniProtKB:Q5HYC2",
  "term_label": "Unknown molecular function",
  "gene_symbol": "KIAA2026",
  "term_id": "UNKNOWN:0001",
  "gene_name": "Uncharacterized protein KIAA2026"
}